{
  "gene": "UniProtKB:Q9UPW6",
  "term_id": "GO:0006338",
  "term_label": "chromatin remodeling",
  "gene_name": "DNA-binding protein SATB2",
  "gene_symbol": "SATB2"
}